icosahedral viral capsid, collar fiber [GO:0098032] (cellular component) Definition: A fiber attached to the collar structure of some icosahedral viral capsids. Sources: GOC:bm Relationships: is a type of GO:0098022; is part of icosahedral viral capsid, collar [GO:0098031]